{
  "term_id": "UNKNOWN:0002",
  "gene": "UniProtKB:Q8WZ92",
  "term_label": "Unknown biological process",
  "gene_symbol": "OR5P2",
  "gene_name": "Olfactory receptor 5P2"
}